{
  "term_label": "nucleus",
  "gene_symbol": "UBE2Q2",
  "gene": "UniProtKB:Q8WVN8",
  "term_id": "GO:0005634",
  "gene_name": "Ubiquitin-conjugating enzyme E2 Q2"
}